{
  "term_label": "clathrin coat assembly",
  "gene": "UniProtKB:P42857",
  "term_id": "GO:0048268",
  "gene_name": "Neuronal vesicle trafficking-associated protein 1",
  "gene_symbol": "NSG1"
}